CAM photosynthesis [GO:0009761] (biological process) Relationships: is a type of GO:0015977; is a type of photosynthesis, dark reaction [GO:0019685] Definition: The combination of atmospheric CO2 with a 3-carbon molecule phosphoenol pyruvate (PEP) to make malic acid. The malic acid is then passed into the vacuole where it is stored until daylight, when it is shuttled back out to be used as a substrate in the light reaction of photosynthesis. Sources: ISBN:0582015952